{
  "gene_symbol": "DUOXA2",
  "term_id": "UNKNOWN:0002",
  "gene": "UniProtKB:Q1HG44",
  "term_label": "Unknown biological process",
  "gene_name": "Dual oxidase maturation factor 2"
}